{
  "gene_symbol": "TMEM177",
  "gene": "UniProtKB:Q53S58",
  "term_label": "membrane",
  "gene_name": "Transmembrane protein 177",
  "term_id": "GO:0016020"
}